{
  "term_id": "GO:0005615",
  "gene_symbol": "RBP4",
  "gene": "UniProtKB:P02753",
  "term_label": "extracellular space",
  "gene_name": "Retinol-binding protein 4"
}